thermospermine biosynthetic process [GO:1903603] (biological process) Definition: The chemical reactions and pathways resulting in the formation of thermospermine. Relationships: is a type of polyamine biosynthetic process [GO:0006596] Also known as: thermospermine anabolism, thermospermine biosynthesis, thermospermine formation, thermospermine synthesis References: PMID:24906355 Sources: GOC:TermGenie, GO_REF:0000068